{
  "term_id": "GO:0015216",
  "term_label": "purine nucleotide transmembrane transporter activity",
  "gene_symbol": "ABCC11",
  "gene": "UniProtKB:Q96J66",
  "gene_name": "ATP-binding cassette sub-family C member 11"
}